Delta14-sterol reductase activity [GO:0050613] (molecular function) Note: Note that zymosterol is cholesta-8,24-dien-3-ol. Definition: Catalysis of the reaction: NADP+ + 4,4-dimethyl-5-alpha-cholesta-8,24-dien-3-beta-ol = NADPH + H+ + 4,4-dimethyl-5-alpha-cholesta-8,14,24-trien-3-beta-ol. Relationships: is a type of oxidoreductase activity, acting on the CH-CH group of donors, NAD or NADP as acceptor [GO:0016628] Also known as: C-14 sterol reductase activity, D14-sterol reductase activity, sterol C-14 reductase activity, 4,4-dimethyl-5alpha-cholesta-8,24-dien-3beta-ol:NADP+ delta14-oxidoreductase activity, sterol C14-reductase activity Sources: EC:1.3.1.70